vacuole-isolation membrane contact site [GO:0120095] (CC) Definition: An organelle membrane contact site formed at the junction of the vacuolar membrane and the isolation membrane or phagophore in response to starvation or other stresses, leading to the formation of the autophagosome. References: PMID:23549786 Also known as: vacuole-IM contact site, vacuole-phagophore contact site, VICS Relationships: is_a GO:0044232